{
  "gene": "UniProtKB:A8K8V0",
  "gene_name": "Zinc finger protein 785",
  "term_label": "DNA-binding transcription factor activity, RNA polymerase II-specific",
  "gene_symbol": "ZNF785",
  "term_id": "GO:0000981"
}